{
  "term_label": "regulation of transcription by RNA polymerase II",
  "term_id": "GO:0006357",
  "gene": "UniProtKB:Q9NPI1",
  "gene_symbol": "BRD7",
  "gene_name": "Bromodomain-containing protein 7"
}